positive regulation of synergid differentiation [GO:0045699] (biological process) Definition: Any process that activates or increases the frequency, rate or extent of synergid cell differentiation. Sources: GOC:go_curators Relationships: is a type of positive regulation of cell differentiation [GO:0045597]; is a type of regulation of synergid differentiation [GO:0045697]; is a type of positive regulation of multicellular organismal process [GO:0051240]; positively regulates synergid differentiation [GO:0009563] Also known as: positive regulation of synergid cell differentiation, up regulation of synergid differentiation, up-regulation of synergid differentiation, upregulation of synergid differentiation, activation of synergid differentiation, stimulation of synergid differentiation